carbamoyl-phosphate synthase (ammonia) activity [GO:0004087] (molecular function) Definition: Catalysis of the reaction: 2 ATP + hydrogencarbonate + NH4+ = 2 ADP + carbamoyl phosphate + 2 H+ + phosphate. Also known as: carbamoyl phosphate synthase (ammonia) activity, CPS I activity, carbamoyl-phosphate synthetase (ammonia) activity, carbamoyl-phosphate synthetase I activity, carbamoylphosphate synthase (ammonia), carbamoylphosphate synthase activity, carbamoylphosphate synthetase (ammonia) activity, carbamylphosphate synthetase I, carbamylphosphate synthetase activity, carbmoylphosphate synthetase activity, carbon-dioxide--ammonia ligase activity, carbon-dioxide:ammonia ligase (ADP-forming, carbamate-phosphorylating) Relationships: is_a ligase activity, forming carbon-nitrogen bonds [GO:0016879] Sources: EC:6.3.4.16, RHEA:18029